{
  "gene_symbol": "ADAMTS9",
  "gene": "UniProtKB:Q9P2N4",
  "gene_name": "A disintegrin and metalloproteinase with thrombospondin motifs 9",
  "term_id": "GO:0006508",
  "term_label": "proteolysis"
}